crossover junction DNA endonuclease activity [GO:0008821] (MF) Definition: Catalysis of the endonucleolytic cleavage at a junction such as a reciprocal single-stranded crossover between two homologous DNA duplexes (Holliday junction). Also known as: crossover junction endodeoxyribonuclease activity, crossover junction endoribonuclease activity, endodeoxyribonuclease RUS activity, Holliday junction endonuclease CCE1 activity, Holliday junction resolvase activity, RusA endonuclease activity, RuvC endonuclease activity, SpCCe1 Holliday junction resolvase activity, SpCCe1 holliday junction resolvase, endonuclease RuvC activity, endonuclease VII activity, endonuclease X3 activity, Hje endonuclease activity, Holliday junction nuclease activity, cruciform-cutting endonuclease activity, endo X3 Relationships: is a type of DNA endonuclease activity, producing 3'-phosphomonoesters [GO:0016889] Sources: EC:3.1.21.10